{
  "term_label": "extracellular space",
  "term_id": "GO:0005615",
  "gene_symbol": "FCGBP",
  "gene_name": "IgGFc-binding protein",
  "gene": "UniProtKB:Q9Y6R7"
}